{
  "term_id": "UNKNOWN:0001",
  "gene": "UniProtKB:Q8N5T2",
  "gene_symbol": "TBC1D19",
  "gene_name": "TBC1 domain family member 19",
  "term_label": "Unknown molecular function"
}